{
  "gene": "UniProtKB:Q96PV6",
  "term_id": "GO:0005634",
  "gene_name": "Leukocyte receptor cluster member 8",
  "gene_symbol": "LENG8",
  "term_label": "nucleus"
}